{
  "term_label": "positive regulation of double-strand break repair via nonhomologous end joining",
  "gene_symbol": "SHLD3",
  "gene": "UniProtKB:Q6ZNX1",
  "gene_name": "Shieldin complex subunit 3",
  "term_id": "GO:2001034"
}